{
  "gene": "UniProtKB:P11362",
  "term_id": "GO:0043410",
  "gene_symbol": "FGFR1",
  "term_label": "positive regulation of MAPK cascade",
  "gene_name": "Fibroblast growth factor receptor 1"
}